{
  "gene_name": "CPX chromosomal region candidate gene 1 protein",
  "gene_symbol": "CPXCR1",
  "term_id": "UNKNOWN:0001",
  "term_label": "Unknown molecular function",
  "gene": "UniProtKB:Q8N123"
}